negative regulation of nucleoside transport [GO:0032243] (biological process) Sources: GOC:mah Subtypes: negative regulation of purine nucleoside transport [GO:0032247] Also known as: down regulation of nucleoside transport, down-regulation of nucleoside transport, downregulation of nucleoside transport, inhibition of nucleoside transport Definition: Any process that stops, prevents, or reduces the frequency, rate or extent of the directed movement of a nucleoside into, out of or within a cell, or between cells, by means of some agent such as a transporter or pore. Relationships: is a type of GO:0032240; is a type of regulation of nucleoside transport [GO:0032242]; negatively regulates nucleoside transport [GO:0015858]